{
  "gene_symbol": "CLDN3",
  "gene_name": "Claudin-3",
  "term_id": "GO:0005923",
  "gene": "UniProtKB:O15551",
  "term_label": "bicellular tight junction"
}